{
  "gene": "UniProtKB:P40429",
  "term_id": "GO:0022625",
  "term_label": "cytosolic large ribosomal subunit",
  "gene_symbol": "RPL13A",
  "gene_name": "Large ribosomal subunit protein uL13"
}